{
  "gene_name": "Ubiquitin carboxyl-terminal hydrolase MINDY-2",
  "gene_symbol": "MINDY2",
  "term_id": "GO:0016807",
  "term_label": "cysteine-type carboxypeptidase activity",
  "gene": "UniProtKB:Q8NBR6"
}